alternative oxidase activity [GO:0009916] (molecular function) Sources: ISBN:0943088399 Definition: Catalysis of the oxidation of ubiquinol by diverting electrons from the standard electron transfer chain, transferring them from ubiquinol to oxygen and generating water as the product. Relationships: is a type of oxidoreductase activity, acting on diphenols and related substances as donors, oxygen as acceptor [GO:0016682]